regulation of methanofuran biosynthetic process [GO:1900351] (biological process) Also known as: regulation of methanofuran biosynthesis Relationships: is a type of regulation of biosynthetic process [GO:0009889]; regulates methanofuran biosynthetic process [GO:2001120] Subtypes: negative regulation of methanofuran biosynthetic process [GO:1900352], GO:1900353 Definition: Any process that modulates the frequency, rate or extent of methanofuran biosynthetic process. Sources: GOC:TermGenie, GOC:mengo_curators